AMP binding [GO:0016208] (molecular function) Relationships: is a type of adenyl ribonucleotide binding [GO:0032559]; is a type of anion binding [GO:0043168]; is a type of cation binding [GO:0043169] Definition: Binding to AMP, adenosine monophosphate. Sources: GOC:go_curators